cycloeucalenol cycloisomerase activity [GO:0047793] (molecular function) Also known as: cycloeucalenol-obtusifoliol isomerase activity, cycloeucalenol lyase (cyclopropane-decyclizing), cycloeucalenol--obtusifoliol isomerase activity Definition: Catalysis of the reaction: cycloeucalenol = obtusifoliol. Relationships: is a type of intramolecular lyase activity [GO:0016872] Sources: EC:5.5.1.9, RHEA:22800